{
  "term_id": "GO:0055037",
  "gene_name": "Putative WAS protein family homolog 4",
  "term_label": "recycling endosome",
  "gene": "UniProtKB:A8MWX3",
  "gene_symbol": "WASH4P"
}